{
  "term_label": "Unknown biological process",
  "gene": "UniProtKB:P11464",
  "gene_name": "Pregnancy-specific beta-1-glycoprotein 1",
  "gene_symbol": "PSG1",
  "term_id": "UNKNOWN:0002"
}